{
  "gene_name": "C-C chemokine receptor type 9",
  "gene": "UniProtKB:P51686",
  "term_id": "GO:0019957",
  "term_label": "C-C chemokine binding",
  "gene_symbol": "CCR9"
}